{
  "gene": "UniProtKB:Q92843",
  "gene_name": "Bcl-2-like protein 2",
  "gene_symbol": "BCL2L2",
  "term_id": "GO:0097192",
  "term_label": "extrinsic apoptotic signaling pathway in absence of ligand"
}